{
  "term_id": "GO:0050431",
  "gene": "UniProtKB:Q8N2S1",
  "gene_name": "Latent-transforming growth factor beta-binding protein 4",
  "gene_symbol": "LTBP4",
  "term_label": "transforming growth factor beta binding"
}